{
  "gene_symbol": "SSH2",
  "term_label": "cytoplasm",
  "term_id": "GO:0005737",
  "gene_name": "Protein phosphatase Slingshot homolog 2",
  "gene": "UniProtKB:Q76I76"
}